{
  "gene": "UniProtKB:Q5JUK9",
  "gene_symbol": "PAGE3",
  "term_id": "UNKNOWN:0001",
  "term_label": "Unknown molecular function",
  "gene_name": "P antigen family member 3"
}